{
  "term_label": "endocytic recycling",
  "gene": "UniProtKB:O75379",
  "gene_symbol": "VAMP4",
  "gene_name": "Vesicle-associated membrane protein 4",
  "term_id": "GO:0032456"
}